{
  "gene_symbol": "CA6",
  "term_label": "extracellular space",
  "gene_name": "Carbonic anhydrase 6",
  "term_id": "GO:0005615",
  "gene": "UniProtKB:P23280"
}